{
  "gene_symbol": "GNAI2",
  "gene_name": "Guanine nucleotide-binding protein G(i) subunit alpha-2",
  "term_label": "adenylate cyclase-inhibiting G protein-coupled receptor signaling pathway",
  "term_id": "GO:0007193",
  "gene": "UniProtKB:P04899"
}